{
  "gene": "UniProtKB:Q8IWU6",
  "gene_name": "Extracellular sulfatase Sulf-1",
  "term_id": "GO:0009986",
  "term_label": "cell surface",
  "gene_symbol": "SULF1"
}